{
  "gene_symbol": "KRT26",
  "gene": "UniProtKB:Q7Z3Y9",
  "gene_name": "Keratin, type I cytoskeletal 26",
  "term_id": "GO:0045109",
  "term_label": "intermediate filament organization"
}